{
  "gene_name": "Prepronociceptin",
  "gene": "UniProtKB:Q13519",
  "gene_symbol": "PNOC",
  "term_id": "GO:0007600",
  "term_label": "sensory perception"
}